{
  "gene_symbol": "RGS14",
  "gene_name": "Regulator of G-protein signaling 14",
  "term_label": "spindle organization",
  "term_id": "GO:0007051",
  "gene": "UniProtKB:O43566"
}